collectin binding [GO:0001862] (molecular function) Sources: GOC:add, ISBN:0781735149 Relationships: is a type of opsonin binding [GO:0001846] Definition: Binding to a collectin, a member of a group of structurally related pattern recognition molecules characterized by having a carbohydrate recognition domain of the C-type lectin family at the C-terminus and a collagenous domain at the N-terminus. Note: Note that collectins include such proteins as mannose-binding lectins (MBL) and surfactant proteins A and D (SP-A and SP-D).